{
  "gene_symbol": "BLVRA",
  "term_id": "UNKNOWN:0002",
  "gene": "UniProtKB:P53004",
  "gene_name": "Biliverdin reductase A",
  "term_label": "Unknown biological process"
}